{
  "gene": "UniProtKB:Q8TEE9",
  "gene_name": "Histone deacetylase complex subunit SAP25",
  "gene_symbol": "SAP25",
  "term_id": "UNKNOWN:0001",
  "term_label": "Unknown molecular function"
}